{
  "gene_symbol": "TIRAP",
  "term_id": "GO:0043123",
  "gene_name": "Toll_interleukin-1 receptor domain-containing adapter protein",
  "term_label": "positive regulation of canonical NF-kappaB signal transduction",
  "gene": "UniProtKB:P58753"
}